Ric1-Rgp1 guanyl-nucleotide exchange factor complex [GO:0034066] (cellular component) References: PMID:10990452 Sources: GOC:jh, GOC:mah Also known as: Ric1p-Rgp1p complex Relationships: is a type of guanyl-nucleotide exchange factor complex [GO:0032045]; is part of Golgi apparatus [GO:0005794] Definition: A protein complex that acts as a nucleotide exchange factor for the GTPase Ypt6p, and is required for fusion of endosome-derived vesicles with the Golgi.